beta-galactosidase activity [GO:0004565] (molecular function) Relationships: is a type of GO:0015925 Definition: Catalysis of the hydrolysis of terminal, non-reducing beta-D-galactose residues in beta-D-galactosides. Regulation: negatively regulated by negative regulation of beta-galactosidase activity [GO:1903770]; positively regulated by positive regulation of beta-galactosidase activity [GO:1903771] Sources: EC:3.2.1.23 Note: Note that the inclusion of 'MetaCyc:BGALACT-PWY' is exceptional: normally MetaCyc pathway entries are database references for biological process terms, not molecular function terms. An exception was made in this case because the MetaCyc entry 'BGALACT-PWY' describes only one reaction, that catalyzed by beta-galactosidase. Also known as: beta-D-galactanase activity, beta-D-galactoside galactohydrolase activity, beta-D-lactosidase activity, beta-lactosidase activity, exo-(1->4)-beta-D-galactanase activity, hydrolact Subtypes: galactan 1,3-beta-galactosidase activity [GO:0033943]